{
  "gene": "UniProtKB:O14526",
  "gene_symbol": "FCHO1",
  "gene_name": "F-BAR domain only protein 1",
  "term_label": "clathrin-dependent endocytosis",
  "term_id": "GO:0072583"
}